{
  "term_label": "regulation of Rho protein signal transduction",
  "term_id": "GO:0035023",
  "gene": "UniProtKB:Q9Y3M8",
  "gene_symbol": "STARD13",
  "gene_name": "StAR-related lipid transfer protein 13"
}